{
  "gene": "UniProtKB:Q6IE38",
  "term_label": "negative regulation of proteolysis",
  "term_id": "GO:0045861",
  "gene_name": "Serine protease inhibitor Kazal-type 14",
  "gene_symbol": "SPINK14"
}